{
  "gene_symbol": "SEC14L2",
  "term_id": "GO:0005829",
  "gene": "UniProtKB:O76054",
  "gene_name": "SEC14-like protein 2",
  "term_label": "cytosol"
}